{
  "term_id": "UNKNOWN:0002",
  "term_label": "Unknown biological process",
  "gene_name": "Sperm protein associated with the nucleus on the X chromosome B1",
  "gene_symbol": "SPANXB1",
  "gene": "UniProtKB:Q9NS25"
}